{
  "gene_symbol": "PRKD2",
  "term_label": "phospholipase C-activating G protein-coupled receptor signaling pathway",
  "term_id": "GO:0007200",
  "gene_name": "Serine_threonine-protein kinase D2",
  "gene": "UniProtKB:Q9BZL6"
}